miRNA-mediated gene silencing by mRNA destabilization [GO:0035279] (biological process) Relationships: is a type of miRNA-mediated post-transcriptional gene silencing [GO:0035195]; is a type of mRNA destabilization [GO:0061157] References: PMID:14744438, PMID:15196554, PMID:21118121, PMID:23209154 Sources: GOC:dph, GOC:mtg_lung Also known as: gene silencing by mRNA cleavage, gene silencing by miRNA, mRNA cleavage, mRNA cleavage involved in gene silencing by miRNA, mRNA cleavage involved in gene silencing by microRNA, mRNA destabilization-mediated gene silencing by miRNA, miRNA-mediated gene silencing, mRNA cleavage, deadenylation involved in gene silencing by miRNA, mRNA deadenylation-mediated gene silencing by miRNA, miRNA-mediated gene silencing by mRNA deadenylation Definition: An RNA interference pathway in which microRNAs (miRNAs) direct the cleavage of target mRNAs. Once incorporated into a RNA-induced silencing complex (RISC), a miRNA base pairing with near-perfect complementarity to the target mRNA will typically direct targeted endonucleolytic cleavage of the mRNA. Many plant miRNAs downregulate gene expression through this mechanism.